{
  "gene_name": "Ribonucleoprotein PTB-binding 2",
  "gene_symbol": "RAVER2",
  "term_label": "RNA binding",
  "gene": "UniProtKB:Q9HCJ3",
  "term_id": "GO:0003723"
}